cellular response to temperature stimulus [GO:0071502] (biological process) Also known as: cellular response to thermal stimulus Sources: GOC:mah Definition: Any process that results in a change in state or activity of a cell (in terms of movement, secretion, enzyme production, gene expression, etc.) as a result of a temperature stimulus. Relationships: is a type of response to temperature stimulus [GO:0009266]